{
  "term_id": "UNKNOWN:0001",
  "gene_name": "Inter-alpha-trypsin inhibitor heavy chain H3",
  "gene": "UniProtKB:Q06033",
  "gene_symbol": "ITIH3",
  "term_label": "Unknown molecular function"
}